L-aspartate catabolic process [GO:0006533] (biological process) Definition: The chemical reactions and pathways resulting in the breakdown of L-aspartate, the anion derived from aspartic acid, 2-aminobutanedioic acid. Sources: GOC:go_curators, ISBN:0198506732 Also known as: aspartate breakdown, aspartate catabolism, aspartate degradation Relationships: is a type of aspartate metabolic process [GO:0006531]; is a type of GO:0043649; is_a L-amino acid catabolic process [GO:0170035]; is_a proteinogenic amino acid catabolic process [GO:0170040]